negative regulation of skeletal muscle satellite cell proliferation [GO:1902723] (biological process) Relationships: is a type of regulation of skeletal muscle satellite cell proliferation [GO:0014842]; is a type of negative regulation of skeletal muscle cell proliferation [GO:0014859]; negatively regulates GO:0014841 References: PMID:23212449 Sources: GOC:TermGenie, GO_REF:0000058 Definition: Any process that stops, prevents or reduces the frequency, rate or extent of satellite cell proliferation. Also known as: down regulation of satellite cell proliferation, down-regulation of satellite cell proliferation, downregulation of satellite cell proliferation, inhibition of satellite cell proliferation Subtypes: negative regulation of growth factor dependent skeletal muscle satellite cell proliferation [GO:1902727]